{
  "term_label": "mucin granule",
  "gene": "UniProtKB:Q9BV40",
  "gene_symbol": "VAMP8",
  "gene_name": "Vesicle-associated membrane protein 8",
  "term_id": "GO:0098594"
}